alpha-copaene catabolic process [GO:1901930] (biological process) References: PMID:22867794 Sources: GOC:TermGenie Also known as: alpha-copaene breakdown, alpha-copaene catabolism, alpha-copaene degradation Relationships: is a type of sesquiterpene catabolic process [GO:0051763] Definition: The chemical reactions and pathways resulting in the breakdown of alpha-copaene.